{
  "gene": "UniProtKB:A0A1W2PPE3",
  "gene_symbol": "C1orf202",
  "gene_name": "Uncharacterized protein C1orf202",
  "term_label": "Unknown cellular component",
  "term_id": "UNKNOWN:0003"
}